{
  "gene_symbol": "TRPV4",
  "term_label": "osmosensory signaling pathway",
  "gene_name": "Transient receptor potential cation channel subfamily V member 4",
  "term_id": "GO:0007231",
  "gene": "UniProtKB:Q9HBA0"
}